{
  "gene": "UniProtKB:O94992",
  "gene_name": "Protein HEXIM1",
  "term_id": "GO:0005654",
  "gene_symbol": "HEXIM1",
  "term_label": "nucleoplasm"
}